{
  "gene": "UniProtKB:P0DTW1",
  "term_label": "Unknown cellular component",
  "gene_name": "G antigen 1",
  "gene_symbol": "GAGE1",
  "term_id": "UNKNOWN:0003"
}